regulation of signal transduction involved in conjugation with cellular fusion [GO:0060238] (biological process) Definition: Any process that modulates the rate, frequency or extent of pheromone-dependent signal transduction during conjugation with cellular fusion. Sources: GOC:dph, GOC:tb Relationships: is a type of GO:0009966; is a type of regulation of conjugation with cellular fusion [GO:0031137]; RO_0002211 signal transduction involved in positive regulation of conjugation with cellular fusion [GO:0032005] Subtypes: GO:0010969, positive regulation of signal transduction involved in conjugation with cellular fusion [GO:0060239], negative regulation of signal transduction involved in conjugation with cellular fusion [GO:0060240]